{
  "term_label": "cytosol",
  "gene_symbol": "EEF1AKMT3",
  "term_id": "GO:0005829",
  "gene": "UniProtKB:Q96AZ1",
  "gene_name": "EEF1A lysine methyltransferase 3"
}